{
  "term_label": "innate immune response",
  "gene_symbol": "RFPL4B",
  "gene_name": "Ret finger protein-like 4B",
  "term_id": "GO:0045087",
  "gene": "UniProtKB:Q6ZWI9"
}